{
  "gene_name": "Ras-related protein Rab-41",
  "gene": "UniProtKB:Q5JT25",
  "gene_symbol": "RAB41",
  "term_label": "retrograde vesicle-mediated transport, Golgi to endoplasmic reticulum",
  "term_id": "GO:0006890"
}